{
  "gene": "UniProtKB:P51812",
  "gene_name": "Ribosomal protein S6 kinase alpha-3",
  "gene_symbol": "RPS6KA3",
  "term_label": "ribosomal protein S6 kinase activity",
  "term_id": "GO:0004711"
}